{
  "term_label": "plasma membrane",
  "term_id": "GO:0005886",
  "gene_name": "Natural cytotoxicity triggering receptor 1",
  "gene_symbol": "NCR1",
  "gene": "UniProtKB:O76036"
}